{
  "term_id": "UNKNOWN:0003",
  "gene": "UniProtKB:Q8WU58",
  "gene_symbol": "FAM222B",
  "term_label": "Unknown cellular component",
  "gene_name": "Protein FAM222B"
}